neuropilin binding [GO:0038191] (molecular function) Relationships: is a type of signaling receptor binding [GO:0005102] Definition: Binding to a member of the neuropilin family. References: PMID:23871893 Sources: GOC:bf Also known as: Nrp binding, neuropilin-binding, Nrp ligand